{
  "term_id": "UNKNOWN:0001",
  "gene_name": "Bone marrow proteoglycan",
  "gene": "UniProtKB:P13727",
  "gene_symbol": "PRG2",
  "term_label": "Unknown molecular function"
}